regulation of cell adhesion mediated by integrin [GO:0033628] (biological process) Also known as: regulation of cell adhesion mediated by integrin complex Subtypes: negative regulation of cell adhesion mediated by integrin [GO:0033629], GO:0033630, GO:0033632 Sources: GOC:add Relationships: is a type of regulation of cell adhesion [GO:0030155]; regulates cell adhesion mediated by integrin [GO:0033627] Definition: Any process that modulates the frequency, rate, or extent of cell adhesion mediated by integrin.